aminoacyltransferase activity [GO:0016755] (molecular function) Subtypes: peptidyltransferase activity [GO:0000048], protein-glutamine gamma-glutamyltransferase activity [GO:0003810], arginyl-tRNA--protein transferase activity [GO:0004057], leucyl-tRNA--protein transferase activity [GO:0008914], glutaminyl-peptide cyclotransferase activity [GO:0016603], glutathione gamma-glutamylcysteinyltransferase activity [GO:0016756], ubiquitin-like protein transferase activity [GO:0019787], UDP-N-acetylmuramoylpentapeptide-lysine N6-alanyltransferase activity [GO:0047206], phosphatidylglycerol alanyltransferase activity [GO:0047637], GO:0047811, D-glutamyltransferase activity [GO:0047823], phosphatidylglycerol lysyltransferase activity [GO:0050071], protein-lysine lysyltransferase activity [GO:0052868], eoxin D4 synthase activity [GO:0097262], hypoglycin A gamma-glutamyl transpeptidase activity [GO:0102953], leukotriene C4 gamma-glutamyl transferase activity [GO:0103068] Relationships: is a type of acyltransferase activity [GO:0016746] Also known as: transferase activity, transferring amino-acyl groups Sources: GOC:jl Definition: Catalysis of the transfer of an amino-acyl group from one compound (donor) to another (acceptor).